{
  "term_label": "intermediate filament",
  "gene_symbol": "EPPK1",
  "gene_name": "Epiplakin",
  "gene": "UniProtKB:P58107",
  "term_id": "GO:0005882"
}